{
  "gene_symbol": "CUL1",
  "term_id": "GO:0031146",
  "gene": "UniProtKB:Q13616",
  "term_label": "SCF-dependent proteasomal ubiquitin-dependent protein catabolic process",
  "gene_name": "Cullin-1"
}